negative regulation of cilium assembly [GO:1902018] (biological process) References: PMID:17719545 Sources: GOC:TermGenie, GOC:cilia, GOC:dph Relationships: is a type of negative regulation of plasma membrane bounded cell projection assembly [GO:0120033]; is a type of regulation of cilium assembly [GO:1902017]; is a type of negative regulation of organelle assembly [GO:1902116]; negatively regulates cilium assembly [GO:0060271] Definition: Any process that stops, prevents or reduces the frequency, rate or extent of cilium assembly. Subtypes: negative regulation of non-motile cilium assembly [GO:1902856], negative regulation of motile cilium assembly [GO:1905504] Also known as: down regulation of ciliogenesis, down regulation of cilium assembly, down-regulation of ciliogenesis, down-regulation of cilium assembly, downregulation of ciliogenesis, downregulation of cilium assembly, inhibition of ciliogenesis, negative regulation of ciliogenesis, inhibition of cilium assembly, down regulation of cilium biogenesis, down-regulation of cilium biogenesis, downregulation of cilium biogenesis, inhibition of cilium biogenesis, negative regulation of cilium biogenesis